{
  "term_id": "GO:0005739",
  "gene": "UniProtKB:Q9Y3A0",
  "term_label": "mitochondrion",
  "gene_symbol": "COQ4",
  "gene_name": "Ubiquinone biosynthesis protein COQ4 homolog, mitochondrial"
}